{
  "gene_name": "Interferon gamma",
  "term_label": "cytokine activity",
  "gene_symbol": "IFNG",
  "gene": "UniProtKB:P01579",
  "term_id": "GO:0005125"
}